{
  "term_id": "GO:0006606",
  "gene_name": "Putative nuclear envelope pore membrane protein POM 121B",
  "gene_symbol": "POM121B",
  "term_label": "protein import into nucleus",
  "gene": "UniProtKB:A6NF01"
}